positive regulation of female receptivity [GO:0045925] (biological process) Definition: Any process that activates or increases the receptiveness of a female to male advances. Sources: GOC:go_curators Subtypes: positive regulation of female receptivity, post-mating [GO:0046009] Relationships: is a type of GO:0045924 Also known as: up regulation of female receptivity, up-regulation of female receptivity, upregulation of female receptivity, activation of female receptivity, stimulation of female receptivity